{
  "gene": "UniProtKB:Q9BY84",
  "gene_name": "Dual specificity protein phosphatase 16",
  "term_label": "MAP kinase tyrosine phosphatase activity",
  "term_id": "GO:0033550",
  "gene_symbol": "DUSP16"
}